{
  "term_label": "guanyl-nucleotide exchange factor activity",
  "gene": "UniProtKB:Q5TH69",
  "gene_name": "Brefeldin A-inhibited guanine nucleotide-exchange protein 3",
  "term_id": "GO:0005085",
  "gene_symbol": "ARFGEF3"
}